all-trans-retinyl-palmitate hydrolase, all-trans-retinol forming activity [GO:0047376] (molecular function) Relationships: is a type of GO:0050253 Sources: RHEA:13933 Also known as: all-trans-retinyl-palmitate acylhydrolase activity, all-trans-retinyl-palmitate hydrolase activity, retinyl-palmitate palmitohydrolase activity Definition: Catalysis of the reaction: all-trans-retinyl palmitate + H2O = all-trans-retinol + H+ + palmitate.